PAN complex [GO:0031251] (cellular component) References: PMID:9774670 Also known as: poly(A) nuclease complex Relationships: is_a GO:1905354; is part of cytoplasm [GO:0005737] Definition: A complex that possesses poly(A)-specific ribonuclease activity; catalyzes the message-specific shortening of mRNA poly(A) tails. Contains at least two subunits, known as Pan2p and Pan3p in Saccharomyces.